{
  "term_id": "GO:0005768",
  "term_label": "endosome",
  "gene": "UniProtKB:Q8NEB9",
  "gene_symbol": "PIK3C3",
  "gene_name": "Phosphatidylinositol 3-kinase catalytic subunit type 3"
}